venom-mediated pore formation in membrane of another organism [GO:0044471] (biological process) Definition: A process that begins with venom being forced into an organism by the bite or sting of another organism, and ends with the aggregation, arrangement and bonding together of a set of components to form a pore complex in a membrane of the bitten organism. References: PMID:21549739 Sources: GOC:fj, GOC:jl Also known as: envenomation resulting in pore formation in membrane of another organism, envenomation resulting in pore formation in membrane of other organism Relationships: is a type of GO:0140138; has part GO:0035915